{
  "gene_name": "Kelch-like protein 1",
  "term_label": "dendrite development",
  "gene": "UniProtKB:Q9NR64",
  "gene_symbol": "KLHL1",
  "term_id": "GO:0016358"
}